{
  "term_label": "regulation of transcription by RNA polymerase II",
  "gene_symbol": "ZNF696",
  "gene": "UniProtKB:Q9H7X3",
  "gene_name": "Zinc finger protein 696",
  "term_id": "GO:0006357"
}